{
  "term_id": "UNKNOWN:0002",
  "gene": "UniProtKB:Q9H8V8",
  "term_label": "Unknown biological process",
  "gene_symbol": "Q9H8V8",
  "gene_name": "Putative uncharacterized protein FLJ13197"
}